{
  "term_label": "dendrite",
  "gene": "UniProtKB:Q99835",
  "gene_symbol": "SMO",
  "term_id": "GO:0030425",
  "gene_name": "Protein smoothened"
}